CGC codon-amino acid adaptor activity [GO:0033430] (molecular function) Note: Note that in the standard genetic code, CGC codes for arginine. Definition: A triplet codon-amino acid adaptor activity that recognizes a CGC codon. Also known as: arginine tRNA Relationships: is a type of triplet codon-amino acid adaptor activity [GO:0030533] Sources: GOC:mah